regulation of lamellipodium organization [GO:1902743] (biological process) Relationships: is a type of regulation of plasma membrane bounded cell projection organization [GO:0120035]; regulates lamellipodium organization [GO:0097581] References: PMID:16054028 Sources: GOC:TermGenie, GOC:als, GO_REF:0000058 Definition: Any process that modulates the frequency, rate or extent of lamellipodium organization. Subtypes: regulation of lamellipodium assembly [GO:0010591], negative regulation of lamellipodium organization [GO:1902744], positive regulation of lamellipodium organization [GO:1902745], regulation of lamellipodium morphogenesis [GO:2000392]